{
  "term_id": "GO:0060326",
  "gene_symbol": "PDGFRB",
  "gene": "UniProtKB:P09619",
  "gene_name": "Platelet-derived growth factor receptor beta",
  "term_label": "cell chemotaxis"
}